{
  "gene_name": "Insulin-like growth factor II",
  "term_label": "positive regulation of activated T cell proliferation",
  "gene_symbol": "IGF2",
  "term_id": "GO:0042104",
  "gene": "UniProtKB:P01344"
}